{
  "term_id": "GO:0030378",
  "term_label": "serine racemase activity",
  "gene_symbol": "SRR",
  "gene": "UniProtKB:Q9GZT4",
  "gene_name": "Serine racemase"
}